{
  "gene": "UniProtKB:P37058",
  "gene_name": "17-beta-hydroxysteroid dehydrogenase type 3",
  "gene_symbol": "HSD17B3",
  "term_label": "steroid biosynthetic process",
  "term_id": "GO:0006694"
}